{
  "term_label": "nucleus",
  "gene_name": "LIM_homeobox protein Lhx9",
  "gene_symbol": "LHX9",
  "gene": "UniProtKB:Q9NQ69",
  "term_id": "GO:0005634"
}